{
  "gene_name": "Alpha-2-antiplasmin",
  "gene": "UniProtKB:P08697",
  "gene_symbol": "SERPINF2",
  "term_label": "serine-type endopeptidase inhibitor activity",
  "term_id": "GO:0004867"
}